negative regulation of growth [GO:0045926] (biological process) Definition: Any process that stops, prevents or reduces the rate or extent of growth, the increase in size or mass of all or part of an organism. Sources: GOC:go_curators Also known as: down regulation of growth, down-regulation of growth, downregulation of growth, inhibition of growth Relationships: is a type of regulation of growth [GO:0040008]; is a type of GO:0048519; negatively regulates growth [GO:0040007] Subtypes: negative regulation of cell growth [GO:0030308], GO:0045967, GO:0048640, GO:0060258, negative regulation of secondary growth [GO:2000604]